{
  "gene_symbol": "PDGFA",
  "term_id": "GO:0030335",
  "term_label": "positive regulation of cell migration",
  "gene": "UniProtKB:P04085",
  "gene_name": "Platelet-derived growth factor subunit A"
}